negative regulation of polyamine transmembrane transport [GO:1902268] (biological process) Definition: Any process that stops, prevents or reduces the frequency, rate or extent of polyamine transmembrane transport. References: PMID:23755272 Sources: GOC:TermGenie Relationships: is_a negative regulation of transmembrane transport [GO:0034763]; is_a regulation of polyamine transmembrane transport [GO:1902267]; negatively regulates polyamine transmembrane transport [GO:1902047] Also known as: down regulation of polyamine transmembrane transport, down-regulation of polyamine transmembrane transport, downregulation of polyamine transmembrane transport, inhibition of polyamine transmembrane transport